{
  "gene": "UniProtKB:Q8NFC6",
  "term_id": "GO:0048188",
  "term_label": "Set1C/COMPASS complex",
  "gene_symbol": "BOD1L1",
  "gene_name": "Biorientation of chromosomes in cell division protein 1-like 1"
}